{
  "gene_name": "RAC-alpha serine_threonine-protein kinase",
  "gene_symbol": "AKT1",
  "term_id": "UNKNOWN:0003",
  "term_label": "Unknown cellular component",
  "gene": "UniProtKB:P31749"
}